{
  "gene_name": "Protein BTG4",
  "gene_symbol": "BTG4",
  "gene": "UniProtKB:Q9NY30",
  "term_id": "GO:0005737",
  "term_label": "cytoplasm"
}